{
  "term_id": "GO:0001782",
  "gene_name": "Serine_threonine-protein phosphatase 2A regulatory subunit B'' subunit gamma",
  "term_label": "B cell homeostasis",
  "gene_symbol": "PPP2R3C",
  "gene": "UniProtKB:Q969Q6"
}